{
  "term_id": "GO:0030674",
  "gene": "UniProtKB:Q9BXP5",
  "term_label": "protein-macromolecule adaptor activity",
  "gene_symbol": "SRRT",
  "gene_name": "Serrate RNA effector molecule homolog"
}